peptidyl-aspartic acid hydroxylation [GO:0042264] (biological process) Also known as: peptidyl-aspartic acid/asparagine hydroxylation Sources: GOC:mah Definition: The hydroxylation of peptidyl-aspartic acid to form peptidyl-hydroxyaspartic acid. Relationships: is a type of protein hydroxylation [GO:0018126]; is a type of peptidyl-aspartic acid modification [GO:0018197]